S-adenosyl-L-methionine lyase activity [GO:0047625] (molecular function) Definition: Catalysis of the reaction: S-adenosyl-L-methionine = L-homoserine lactone + S-methyl-5'-thioadenosine. Sources: RHEA:21932 Also known as: SAM lyase activity, adenosyl methionine cyclotransferase activity, adenosylmethionine cyclotransferase activity, S-adenosyl-L-methionine alkyltransferase (cyclizing) activity Relationships: is a type of carbon-sulfur lyase activity [GO:0016846]